{
  "gene": "UniProtKB:A6NCF6",
  "gene_name": "Putative MAGE domain-containing protein MAGEA13P",
  "gene_symbol": "MAGEA13P",
  "term_label": "nucleus",
  "term_id": "GO:0005634"
}